{
  "gene_symbol": "CYRIB",
  "term_id": "UNKNOWN:0003",
  "gene": "UniProtKB:Q9NUQ9",
  "term_label": "Unknown cellular component",
  "gene_name": "CYFIP-related Rac1 interactor B"
}